neural plate elongation [GO:0014022] (biological process) Definition: The process in which the neural plate is shaped by the intrinsic movement of the epidermal and neural plate regions. Sources: GOC:ef, ISBN:0878932585 Relationships: is a type of morphogenesis of an epithelial sheet [GO:0002011]; is_a GO:0048598; is part of GO:0001839